{
  "gene_name": "Kin of IRRE-like protein 1",
  "term_id": "GO:0005911",
  "term_label": "cell-cell junction",
  "gene_symbol": "KIRREL1",
  "gene": "UniProtKB:Q96J84"
}